{
  "gene": "UniProtKB:Q8N5Y2",
  "term_id": "GO:0072487",
  "term_label": "MSL complex",
  "gene_name": "Male-specific lethal 3 homolog",
  "gene_symbol": "MSL3"
}